{
  "term_id": "GO:0031123",
  "gene_name": "Terminal nucleotidyltransferase 4B",
  "term_label": "RNA 3'-end processing",
  "gene_symbol": "TENT4B",
  "gene": "UniProtKB:Q8NDF8"
}